{
  "term_label": "Unknown molecular function",
  "term_id": "UNKNOWN:0001",
  "gene_symbol": "MICOS13",
  "gene": "UniProtKB:Q5XKP0",
  "gene_name": "MICOS complex subunit MIC13"
}